{
  "gene_symbol": "ANAPC1",
  "term_id": "GO:0031145",
  "gene_name": "Anaphase-promoting complex subunit 1",
  "term_label": "anaphase-promoting complex-dependent catabolic process",
  "gene": "UniProtKB:Q9H1A4"
}